inductive cell-cell signaling [GO:0031129] (biological process) Definition: Signaling at short range between cells of different ancestry and developmental potential that results in one cell or group of cells effecting a developmental change in the other. This is often done by secretion of proteins by one cell which affects the neighboring cells and causes them to adopt a certain fate. Subtypes: inductive cell-cell signaling between paraxial mesoderm and motor neuron precursors [GO:0021916], GO:0060494, inductive mesenchymal to epithelial cell signaling [GO:0060522] Relationships: is a type of developmental induction [GO:0031128] Also known as: inductive cell-cell signalling Sources: GOC:mah